{
  "gene_symbol": "NRP1",
  "gene": "UniProtKB:O14786",
  "term_id": "GO:0001755",
  "gene_name": "Neuropilin-1",
  "term_label": "neural crest cell migration"
}